multiple synapse bouton [GO:0150086] (cellular component) Relationships: is a type of terminal bouton [GO:0043195] Also known as: MSB, multi-synapse bouton, multi-synaptic bouton, multiple spine synapse bouton, multiple-synapse bouton, multisynapse bouton, multisynaptic bouton, multi-synapse, multiple synapse, multisynapse Subtypes: GO:0150087, multiple synapse bouton, contacting multiple dendrites [GO:0150088] Definition: A single axon terminal bouton making contact onto two or more dendritic spines protruding either from a single dendrite or from multiple dendrites. References: PMID:10586883, PMID:11248111, PMID:11466428, PMID:18501438, PMID:22028887, PMID:29774619, PMID:7482800, PMID:8366344 Sources: GOC:aruk, GOC:bc